{
  "term_id": "GO:0005811",
  "gene_symbol": "ADIG",
  "term_label": "lipid droplet",
  "gene_name": "Adipogenin",
  "gene": "UniProtKB:Q0VDE8"
}